{
  "gene_name": "Putative uncharacterized protein MED14OS",
  "term_label": "Unknown molecular function",
  "term_id": "UNKNOWN:0001",
  "gene": "UniProtKB:P0DP75",
  "gene_symbol": "MED14OS"
}